lymphotoxin complex [GO:0062048] (cellular component) Definition: A homo- or heterotrimeric protein containing complex consisting of alpha and beta lymphotoxin subunits in different stoichiometric combinations. Also known as: lymphotoxin alpha-beta References: PMID:1733951 Relationships: is a type of protein-containing complex [GO:0032991]